{
  "term_label": "fatty acid elongation, polyunsaturated fatty acid",
  "gene": "UniProtKB:Q9HB03",
  "term_id": "GO:0034626",
  "gene_symbol": "ELOVL3",
  "gene_name": "Elongation of very long chain fatty acids protein 3"
}